vesicle fusion with Golgi apparatus [GO:0048280] (biological process) Sources: GOC:jid Relationships: is a type of GO:0006906; is_a GO:0007030; is part of Golgi vesicle transport [GO:0048193] Definition: The joining of the lipid bilayer membrane around a vesicle to the lipid bilayer membrane around the Golgi. Regulation: regulated by regulation of vesicle fusion with Golgi apparatus [GO:0106214]; negatively regulated by GO:0106215; positively regulated by positive regulation of vesicle fusion with Golgi apparatus [GO:0106216] Subtypes: vesicle fusion with Golgi medial cisterna membrane [GO:1990671], medial-Golgi-derived vesicle fusion with Golgi trans cisterna membrane [GO:1990672], endoplasmic reticulum-Golgi intermediate compartment (ERGIC) derived vesicle fusion with Golgi cis cisterna membrane [GO:1990689], Golgi medial cisterna-derived vesicle fusion with Golgi cis cisterna membrane [GO:1990690], cis-Golgi-derived vesicle fusion with Golgi medial cisterna membrane [GO:1990691], trans-Golgi-derived vesicle fusion with Golgi medial cisterna membrane [GO:1990692]